{
  "gene_name": "ATP-dependent RNA helicase DDX24",
  "gene": "UniProtKB:Q9GZR7",
  "term_id": "GO:0005730",
  "gene_symbol": "DDX24",
  "term_label": "nucleolus"
}